{
  "term_id": "GO:0003823",
  "gene_name": "Immunoglobulin heavy variable 3-73",
  "gene_symbol": "IGHV3-73",
  "gene": "UniProtKB:A0A0B4J1V6",
  "term_label": "antigen binding"
}